{
  "term_id": "GO:0000976",
  "term_label": "transcription cis-regulatory region binding",
  "gene_symbol": "ZNF208",
  "gene": "UniProtKB:O43345",
  "gene_name": "Zinc finger protein 208"
}